{
  "gene_name": "Putative WAS protein family homolog 4",
  "gene_symbol": "WASH4P",
  "term_id": "GO:0032456",
  "gene": "UniProtKB:A8MWX3",
  "term_label": "endocytic recycling"
}